{
  "term_label": "transcription cis-regulatory region binding",
  "gene_name": "Zinc finger protein 658B",
  "gene": "UniProtKB:Q4V348",
  "term_id": "GO:0000976",
  "gene_symbol": "ZNF658B"
}